{
  "term_label": "Arp2/3 complex binding",
  "gene_name": "WASP homolog-associated protein with actin, membranes and microtubules",
  "gene_symbol": "WHAMM",
  "gene": "UniProtKB:Q8TF30",
  "term_id": "GO:0071933"
}